{
  "term_id": "UNKNOWN:0001",
  "gene_name": "Monocyte to macrophage differentiation factor 2",
  "gene_symbol": "MMD2",
  "term_label": "Unknown molecular function",
  "gene": "UniProtKB:Q8IY49"
}